{
  "term_label": "calcium/calmodulin-dependent protein kinase activity",
  "term_id": "GO:0004683",
  "gene_symbol": "MKNK2",
  "gene_name": "MAP kinase-interacting serine_threonine-protein kinase 2",
  "gene": "UniProtKB:Q9HBH9"
}